{
  "term_id": "GO:0006511",
  "gene_symbol": "HERPUD1",
  "term_label": "ubiquitin-dependent protein catabolic process",
  "gene": "UniProtKB:Q15011",
  "gene_name": "Homocysteine-responsive endoplasmic reticulum-resident ubiquitin-like domain member 1 protein"
}